neuroblast fate determination [GO:0007400] (biological process) Also known as: neuroblast cell fate determination, neuroblast identity determination Definition: The cell fate determination process in which a cell becomes capable of differentiating autonomously into a neuroblast cell regardless of its environment; upon determination, the cell fate cannot be reversed. An example of this process is found in Mus musculus. Relationships: is a type of cell fate determination [GO:0001709]; is part of GO:0014017 Sources: GOC:go_curators